{
  "term_id": "GO:0005886",
  "gene": "UniProtKB:P51178",
  "gene_symbol": "PLCD1",
  "term_label": "plasma membrane",
  "gene_name": "1-phosphatidylinositol 4,5-bisphosphate phosphodiesterase delta-1"
}